{
  "gene_symbol": "HGFAC",
  "term_label": "extracellular space",
  "gene_name": "Hepatocyte growth factor activator",
  "term_id": "GO:0005615",
  "gene": "UniProtKB:Q04756"
}